{
  "term_id": "GO:0140374",
  "term_label": "antiviral innate immune response",
  "gene": "UniProtKB:Q9H8X9",
  "gene_symbol": "ZDHHC11",
  "gene_name": "Palmitoyltransferase ZDHHC11"
}